{
  "term_label": "Unknown molecular function",
  "gene_symbol": "LECT2",
  "gene": "UniProtKB:O14960",
  "term_id": "UNKNOWN:0001",
  "gene_name": "Leukocyte cell-derived chemotaxin-2"
}